{
  "term_id": "GO:0043488",
  "term_label": "regulation of mRNA stability",
  "gene_symbol": "FXR2",
  "gene_name": "RNA-binding protein FXR2",
  "gene": "UniProtKB:P51116"
}